{
  "gene_symbol": "ABHD18",
  "term_label": "Unknown biological process",
  "gene": "UniProtKB:Q0P651",
  "gene_name": "Protein ABHD18",
  "term_id": "UNKNOWN:0002"
}